chitin-based cuticle sclerotization [GO:0007593] (biological process) Relationships: is a type of molting cycle, chitin-based cuticle [GO:0007591]; is a type of developmental maturation [GO:0021700]; is a type of molting cycle process [GO:0022404] Definition: The process of hardening of a chitin-based cuticle. Subtypes: GO:0036340, chitin-based cuticle sclerotization by protein cross-linking [GO:0036341] Sources: GOC:dos, GOC:mtg_sensu Regulation: regulated by GO:0007564; negatively regulated by negative regulation of chitin-based cuticle tanning [GO:0045800]; positively regulated by positive regulation of chitin-based cuticle tanning [GO:0045801] Also known as: cuticle hardening, chitin-based cuticle tanning